nitric oxide reductase activity [GO:0016966] (MF) Definition: Catalysis of the reaction: H2O + 2 ferricytochrome c + nitrous oxide = 2 H+ + 2 ferrocytochrome c + 2 nitric oxide. Relationships: is a type of oxidoreductase activity, acting on other nitrogenous compounds as donors, cytochrome as acceptor [GO:0016662] Sources: EC:1.7.2.5 Also known as: CYP55, P450 nitric oxide reductase activity, P450nor, cytochrome bc nitric oxide reductase activity, nitric-oxide reductase activity, nitrogen oxide reductase activity, nitrous-oxide:(acceptor) oxidoreductase (NO-forming), nitrous-oxide:acceptor oxidoreductase (NO-forming)